{
  "term_label": "thermoception",
  "gene_symbol": "TRPM8",
  "gene": "UniProtKB:Q7Z2W7",
  "term_id": "GO:0050955",
  "gene_name": "Transient receptor potential cation channel subfamily M member 8"
}